{
  "gene_name": "Protein FAM118B",
  "gene_symbol": "FAM118B",
  "term_id": "UNKNOWN:0001",
  "term_label": "Unknown molecular function",
  "gene": "UniProtKB:Q9BPY3"
}